{
  "gene": "UniProtKB:Q15572",
  "term_id": "UNKNOWN:0002",
  "term_label": "Unknown biological process",
  "gene_name": "TATA box-binding protein-associated factor RNA polymerase I subunit C",
  "gene_symbol": "TAF1C"
}